{
  "term_label": "protein processing",
  "gene": "UniProtKB:P57727",
  "term_id": "GO:0016485",
  "gene_name": "Transmembrane protease serine 3",
  "gene_symbol": "TMPRSS3"
}